{
  "gene_name": "Solute carrier family 25 member 53",
  "term_id": "UNKNOWN:0002",
  "term_label": "Unknown biological process",
  "gene": "UniProtKB:Q5H9E4",
  "gene_symbol": "SLC25A53"
}